D-glutaminase activity [GO:0050001] (molecular function) Relationships: is a type of hydrolase activity, acting on carbon-nitrogen (but not peptide) bonds, in linear amides [GO:0016811] Also known as: D-glutamine amidohydrolase activity Sources: EC:3.5.1.35, MetaCyc:D-GLUTAMINASE-RXN Definition: Catalysis of the reaction: H2O + L-glutamine = NH3 + D-glutamate.